isoflavonoid phytoalexin catabolic process [GO:0046290] (biological process) Sources: GOC:ai Definition: The chemical reactions and pathways resulting in the breakdown of isoflavonoid phytoalexins, a group of water-soluble phenolic derivatives isomeric with flavonoids that possess antibiotic activity and are produced by plant tissues in response to infection. Relationships: is a type of isoflavonoid catabolic process [GO:0046288]; is a type of phytoalexin catabolic process [GO:0052316] Also known as: isoflavonoid phytoalexin breakdown, isoflavonoid phytoalexin catabolism, isoflavonoid phytoalexin degradation